regulation of methane biosynthetic process from dimethylamine [GO:1900318] (BP) Sources: GOC:TermGenie, GOC:mengo_curators Subtypes: negative regulation of methane biosynthetic process from dimethylamine [GO:1900319], GO:1900320 Definition: Any process that modulates the frequency, rate or extent of methane biosynthetic process from dimethylamine. Relationships: is a type of regulation of amine metabolic process [GO:0033238]; is a type of regulation of cellular respiration [GO:0043457]; is_a GO:1901577; regulates methane biosynthetic process from dimethylamine [GO:2001129]